fructan biosynthetic process [GO:0010146] (biological process) Sources: GOC:pz Relationships: is a type of polysaccharide biosynthetic process [GO:0000271] Also known as: fructan anabolism, fructan biosynthesis, fructan formation, fructan synthesis, levan biosynthesis, levan biosynthetic process Definition: The chemical reactions and pathways resulting in the formation of fructan a polysaccharide consisting of fructose residues. Subtypes: inulin biosynthetic process [GO:1902928]